{
  "gene_name": "Clarin-3",
  "gene": "UniProtKB:Q8NCR9",
  "term_id": "UNKNOWN:0002",
  "gene_symbol": "CLRN3",
  "term_label": "Unknown biological process"
}